plastoquinol--plastocyanin reductase activity [GO:0009496] (molecular function) Relationships: is a type of GO:0009055; is a type of oxidoreduction-driven active transmembrane transporter activity [GO:0015453]; is a type of oxidoreductase activity, acting on diphenols and related substances as donors, with copper protein as acceptor [GO:0052880] Sources: RHEA:22148 Also known as: cytochrome b6f, cytochrome b6f complex activity, plastoquinol-plastocyanin reductase activity, plastoquinol/plastocyanin oxidoreductase activity, plastoquinol:oxidized-plastocyanin oxidoreductase activity Definition: Catalysis of the reaction: 2 H+[side 1] + 2 oxidized plastocyanin + plastoquinol-1 = 2 H+[side 2] + 2 reduced plastocyanin + plastoquinone. This reaction involves the concomitant transfer of 2 H+ ions across a membrane.